{
  "gene_name": "Nuclear receptor-binding protein",
  "gene": "UniProtKB:Q9UHY1",
  "term_id": "GO:0006974",
  "gene_symbol": "NRBP1",
  "term_label": "DNA damage response"
}